{
  "term_label": "SUMO transferase activity",
  "term_id": "GO:0019789",
  "gene": "UniProtKB:A8MTL3",
  "gene_name": "RING finger protein 212B",
  "gene_symbol": "RNF212B"
}